{
  "term_label": "cell-cell signaling",
  "gene_symbol": "FGFBP3",
  "term_id": "GO:0007267",
  "gene_name": "Fibroblast growth factor-binding protein 3",
  "gene": "UniProtKB:Q8TAT2"
}